{
  "gene": "UniProtKB:Q86XT2",
  "term_label": "Unknown molecular function",
  "term_id": "UNKNOWN:0001",
  "gene_name": "Vacuolar protein sorting-associated protein 37D",
  "gene_symbol": "VPS37D"
}